membrane bone morphogenesis [GO:0061973] (biological process) References: PMID:14579374 Definition: The process in which bone which forms deep in the organism are generated and organized. Relationships: is a type of bone morphogenesis [GO:0060349] Subtypes: GO:0061972, perichondral bone morphogenesis [GO:0061974]